{
  "gene_symbol": "NDRG2",
  "term_id": "GO:0005737",
  "gene_name": "Protein NDRG2",
  "gene": "UniProtKB:Q9UN36",
  "term_label": "cytoplasm"
}